{
  "term_id": "GO:0061608",
  "term_label": "nuclear import signal receptor activity",
  "gene": "UniProtKB:Q96P70",
  "gene_name": "Importin-9",
  "gene_symbol": "IPO9"
}